{
  "gene_name": "Threonylcarbamoyl-AMP synthase",
  "gene": "UniProtKB:Q86U90",
  "term_id": "GO:0006450",
  "gene_symbol": "YRDC",
  "term_label": "regulation of translational fidelity"
}